{
  "term_label": "phospholipase C-activating G protein-coupled receptor signaling pathway",
  "gene": "UniProtKB:Q6DWJ6",
  "gene_symbol": "GPR139",
  "gene_name": "Probable G-protein coupled receptor 139",
  "term_id": "GO:0007200"
}